positive regulation of gibberellin biosynthetic process [GO:0010372] (biological process) Also known as: positive regulation of gibberellic acid biosynthetic process Sources: GOC:tair_curators Definition: Any process that activates, maintains or increases the frequency, rate or extent of the chemical reactions and pathways resulting in the formation of gibberellins. Relationships: is a type of regulation of gibberellin biosynthetic process [GO:0010371]; is a type of positive regulation of lipid biosynthetic process [GO:0046889]; is a type of positive regulation of small molecule metabolic process [GO:0062013]; positively regulates gibberellin biosynthetic process [GO:0009686]